sulfur compound transmembrane transporter activity [GO:1901682] (molecular function) Sources: GOC:TermGenie, GOC:pr Relationships: is a type of transmembrane transporter activity [GO:0022857] Definition: Enables the transfer of a sulfur compound from one side of a membrane to the other. Also known as: sulfur molecular entity transmembrane transporter activity Subtypes: GO:0000095, GO:0000099, S-methylmethionine transmembrane transporter activity [GO:0000100], sulfite transmembrane transporter activity [GO:0000319], taurine transmembrane transporter activity [GO:0005368], GO:0008521, sulfate transmembrane transporter activity [GO:0015116], thiosulfate transmembrane transporter activity [GO:0015117], biotin transmembrane transporter activity [GO:0015225], coenzyme A transmembrane transporter activity [GO:0015228], thiamine transmembrane transporter activity [GO:0015234], ABC-type glutathione S-conjugate transporter activity [GO:0015431], GO:0015546, GO:0015607, GO:0034634, ABC-type alkanesulfonate transporter transporter activity [GO:0042959], 3'-phosphoadenosine 5'-phosphosulfate transmembrane transporter activity [GO:0046964], glucosinolate transmembrane transporter activity [GO:0141165], GO:1902557